{
  "gene": "UniProtKB:P63162",
  "term_label": "mRNA splicing, via spliceosome",
  "term_id": "GO:0000398",
  "gene_name": "Small nuclear ribonucleoprotein-associated protein N",
  "gene_symbol": "SNRPN"
}